{
  "gene": "UniProtKB:Q08AM6",
  "term_id": "GO:0006661",
  "term_label": "phosphatidylinositol biosynthetic process",
  "gene_symbol": "VAC14",
  "gene_name": "Protein VAC14 homolog"
}